{
  "term_label": "regulation of transcription by RNA polymerase II",
  "term_id": "GO:0006357",
  "gene_symbol": "SOHLH2",
  "gene_name": "Spermatogenesis- and oogenesis-specific basic helix-loop-helix-containing protein 2",
  "gene": "UniProtKB:Q9NX45"
}